{
  "gene_name": "Putative uncharacterized protein B3GALT5-AS1",
  "term_label": "Unknown molecular function",
  "gene": "UniProtKB:P59052",
  "gene_symbol": "B3GALT5-AS1",
  "term_id": "UNKNOWN:0001"
}